{
  "term_id": "UNKNOWN:0001",
  "term_label": "Unknown molecular function",
  "gene": "UniProtKB:Q58FG1",
  "gene_symbol": "HSP90AA4P",
  "gene_name": "Putative heat shock protein HSP 90-alpha A4"
}